{
  "gene_name": "Nuclear envelope phosphatase-regulatory subunit 1",
  "gene": "UniProtKB:Q8N9A8",
  "term_label": "Nem1-Spo7 phosphatase complex",
  "gene_symbol": "CNEP1R1",
  "term_id": "GO:0071595"
}